{
  "term_label": "AMP kinase activity",
  "term_id": "GO:0004017",
  "gene_symbol": "AK8",
  "gene_name": "Adenylate kinase 8",
  "gene": "UniProtKB:Q96MA6"
}